{
  "gene_symbol": "UGT1A10",
  "term_label": "liver development",
  "gene": "UniProtKB:Q9HAW8",
  "term_id": "GO:0001889",
  "gene_name": "UDP-glucuronosyltransferase 1A10"
}